{
  "gene_symbol": "HESX1",
  "term_label": "regulation of transcription by RNA polymerase II",
  "gene": "UniProtKB:Q9UBX0",
  "term_id": "GO:0006357",
  "gene_name": "Homeobox expressed in ES cells 1"
}